{
  "gene": "UniProtKB:Q86YW7",
  "term_label": "hormone activity",
  "gene_name": "Glycoprotein hormone beta-5",
  "term_id": "GO:0005179",
  "gene_symbol": "GPHB5"
}